{
  "term_label": "Unknown cellular component",
  "gene_name": "Protein LRATD1",
  "gene": "UniProtKB:Q96KN4",
  "gene_symbol": "LRATD1",
  "term_id": "UNKNOWN:0003"
}